{
  "term_id": "UNKNOWN:0002",
  "term_label": "Unknown biological process",
  "gene_name": "HERV-H LTR-associating protein 3",
  "gene_symbol": "HHLA3",
  "gene": "UniProtKB:Q9XRX5"
}